{
  "gene_name": "Zinc finger protein 195",
  "gene_symbol": "ZNF195",
  "term_id": "GO:0006355",
  "gene": "UniProtKB:O14628",
  "term_label": "regulation of DNA-templated transcription"
}